host cell Golgi membrane [GO:0044178] (cellular component) Definition: The lipid bilayer surrounding any of the compartments of the host cell Golgi apparatus. Also known as: host Golgi membrane Sources: GOC:jl Relationships: is a type of host cell membrane [GO:0033644]; is part of GO:0033645; is part of host cell Golgi apparatus [GO:0044177]